{
  "term_id": "GO:0005739",
  "term_label": "mitochondrion",
  "gene_name": "Histatin-3",
  "gene_symbol": "HTN3",
  "gene": "UniProtKB:P15516"
}